{
  "term_label": "cell surface receptor signaling pathway",
  "term_id": "GO:0007166",
  "gene_symbol": "PECAM1",
  "gene_name": "Platelet endothelial cell adhesion molecule",
  "gene": "UniProtKB:P16284"
}